{
  "gene_symbol": "ZKSCAN1",
  "term_id": "GO:0000978",
  "term_label": "RNA polymerase II cis-regulatory region sequence-specific DNA binding",
  "gene_name": "Zinc finger protein with KRAB and SCAN domains 1",
  "gene": "UniProtKB:P17029"
}